{
  "gene_symbol": "LINC01551",
  "gene_name": "Uncharacterized protein encoded by LINC01551",
  "gene": "UniProtKB:Q86U37",
  "term_label": "Unknown cellular component",
  "term_id": "UNKNOWN:0003"
}